{
  "gene": "UniProtKB:Q9UN42",
  "term_label": "Unknown molecular function",
  "gene_name": "Protein ATP1B4",
  "term_id": "UNKNOWN:0001",
  "gene_symbol": "ATP1B4"
}